{
  "gene_symbol": "MS4A6A",
  "gene": "UniProtKB:Q9H2W1",
  "term_id": "GO:0007166",
  "gene_name": "Membrane-spanning 4-domains subfamily A member 6A",
  "term_label": "cell surface receptor signaling pathway"
}